{
  "term_id": "GO:0051015",
  "gene_name": "Macrophage-capping protein",
  "gene_symbol": "CAPG",
  "gene": "UniProtKB:P40121",
  "term_label": "actin filament binding"
}